{
  "term_id": "GO:0003713",
  "gene_symbol": "KMT2D",
  "gene_name": "Histone-lysine N-methyltransferase 2D",
  "gene": "UniProtKB:O14686",
  "term_label": "transcription coactivator activity"
}